{
  "term_label": "nucleus",
  "gene": "UniProtKB:Q13472",
  "term_id": "GO:0005634",
  "gene_name": "DNA topoisomerase 3-alpha",
  "gene_symbol": "TOP3A"
}